{
  "term_id": "UNKNOWN:0002",
  "term_label": "Unknown biological process",
  "gene": "UniProtKB:A0A8I5KXM2",
  "gene_name": "Uncharacterized protein",
  "gene_symbol": "A0A8I5KXM2"
}